{
  "gene": "UniProtKB:P08195",
  "gene_symbol": "SLC3A2",
  "term_id": "GO:0016324",
  "term_label": "apical plasma membrane",
  "gene_name": "4F2 cell-surface antigen heavy chain"
}